endocytic recycling [GO:0032456] (BP) Regulation: regulated by GO:2001135; negatively regulated by GO:2001136; positively regulated by positive regulation of endocytic recycling [GO:2001137] References: PMID:16473635, PMID:23563491 Subtypes: fast endocytic recycling [GO:0032457], slow endocytic recycling [GO:0032458], endosome to plasma membrane protein transport [GO:0099638] Also known as: retrograde transport, endosome to plasma membrane, retrograde transport of endocytic vesicles Definition: The directed movement of membrane-bounded vesicles from endosomes back to the plasma membrane, a trafficking pathway that promotes the recycling of internalized transmembrane proteins. Relationships: is a type of endosomal transport [GO:0016197]; is a type of GO:0098876